{
  "gene": "UniProtKB:Q96QH8",
  "gene_symbol": "SPACA5",
  "term_label": "fusion of sperm to egg plasma membrane involved in single fertilization",
  "gene_name": "Sperm acrosome-associated protein 5",
  "term_id": "GO:0007342"
}